{
  "term_id": "GO:0043161",
  "gene_symbol": "PSMB7",
  "gene": "UniProtKB:Q99436",
  "term_label": "proteasome-mediated ubiquitin-dependent protein catabolic process",
  "gene_name": "Proteasome subunit beta type-7"
}